{
  "gene_name": "Patatin-like phospholipase domain-containing protein 5",
  "term_id": "GO:0005811",
  "gene": "UniProtKB:Q7Z6Z6",
  "term_label": "lipid droplet",
  "gene_symbol": "PNPLA5"
}